{
  "gene_name": "MAPK_MAK_MRK overlapping kinase",
  "term_id": "GO:0035556",
  "gene_symbol": "MOK",
  "term_label": "intracellular signal transduction",
  "gene": "UniProtKB:Q9UQ07"
}